{
  "term_id": "UNKNOWN:0001",
  "gene_symbol": "DEFB124",
  "gene": "UniProtKB:Q8NES8",
  "term_label": "Unknown molecular function",
  "gene_name": "Beta-defensin 124"
}